neural crest cell differentiation [GO:0014033] (biological process) Sources: GOC:dh, GOC:ef Subtypes: cardiac neural crest cell differentiation involved in heart development [GO:0061307], GO:1902637, neural crest cell differentiation involved in parathyroid gland development [GO:1902638] Definition: The process in which a relatively unspecialized cell acquires specialized features of a neural crest cell. Regulation: regulated by GO:1905292; negatively regulated by negative regulation of neural crest cell differentiation [GO:1905293]; positively regulated by GO:1905294 Relationships: is a type of GO:0048762; is a type of stem cell differentiation [GO:0048863]